{
  "gene_name": "Claudin-12",
  "gene": "UniProtKB:P56749",
  "term_label": "plasma membrane",
  "term_id": "GO:0005886",
  "gene_symbol": "CLDN12"
}